respiratory burst involved in inflammatory response [GO:0002536] (biological process) Relationships: is a type of GO:0002532; is a type of respiratory burst involved in defense response [GO:0002679] Regulation: regulated by GO:0060264; positively regulated by positive regulation of respiratory burst involved in inflammatory response [GO:0060265]; negatively regulated by negative regulation of respiratory burst involved in inflammatory response [GO:0060266] Definition: A phase of elevated metabolic activity, during which oxygen consumption increases following a stimulus as part of an inflammatory response; this leads to the production, by an NADH dependent system, of hydrogen peroxide (H2O2), superoxide anions and hydroxyl radicals, resulting in an increase in their intracellular or extracellular levels. Sources: GOC:add, ISBN:0781735149 Also known as: oxidative burst during acute inflammatory response, production of reactive oxygen species during acute inflammatory response, respiratory burst involved in acute inflammatory response